{
  "gene_symbol": "SOX4",
  "gene": "UniProtKB:Q06945",
  "gene_name": "Transcription factor SOX-4",
  "term_label": "DNA-binding transcription activator activity, RNA polymerase II-specific",
  "term_id": "GO:0001228"
}